{
  "gene": "UniProtKB:Q9Y6M7",
  "term_id": "GO:0015701",
  "gene_symbol": "SLC4A7",
  "gene_name": "Sodium bicarbonate cotransporter 3",
  "term_label": "bicarbonate transport"
}